{
  "gene_symbol": "KCTD21",
  "gene": "UniProtKB:Q4G0X4",
  "gene_name": "BTB_POZ domain-containing protein KCTD21",
  "term_id": "GO:0042826",
  "term_label": "histone deacetylase binding"
}